{
  "gene_name": "Rho-related GTP-binding protein RhoN",
  "gene": "UniProtKB:P52198",
  "gene_symbol": "RND2",
  "term_label": "protein kinase binding",
  "term_id": "GO:0019901"
}